{
  "gene": "UniProtKB:Q8IYR0",
  "gene_name": "Cilia- and flagella-associated protein 206",
  "term_label": "ciliary basal body",
  "gene_symbol": "CFAP206",
  "term_id": "GO:0036064"
}